{
  "gene": "UniProtKB:O60248",
  "term_label": "positive regulation of transcription by RNA polymerase II",
  "gene_name": "Protein SOX-15",
  "gene_symbol": "SOX15",
  "term_id": "GO:0045944"
}